{
  "gene_name": "Actin-related protein 2_3 complex subunit 5",
  "term_label": "cell migration",
  "gene_symbol": "ARPC5",
  "gene": "UniProtKB:O15511",
  "term_id": "GO:0016477"
}